{
  "term_label": "nuclear-transcribed mRNA poly(A) tail shortening",
  "gene_symbol": "PAN3",
  "term_id": "GO:0000289",
  "gene_name": "PAN2-PAN3 deadenylation complex subunit PAN3",
  "gene": "UniProtKB:Q58A45"
}